{
  "gene_name": "Periplakin",
  "gene_symbol": "PPL",
  "gene": "UniProtKB:O60437",
  "term_label": "membrane",
  "term_id": "GO:0016020"
}